{
  "term_label": "plasma membrane",
  "gene_symbol": "KIAA0319",
  "gene_name": "Dyslexia-associated protein KIAA0319",
  "gene": "UniProtKB:Q5VV43",
  "term_id": "GO:0005886"
}